{
  "gene_symbol": "TMSB4Y",
  "gene_name": "Thymosin beta-4, Y-chromosomal",
  "term_label": "cytosol",
  "term_id": "GO:0005829",
  "gene": "UniProtKB:O14604"
}